{
  "term_id": "GO:0008349",
  "term_label": "MAP kinase kinase kinase kinase activity",
  "gene": "UniProtKB:Q9Y4K4",
  "gene_name": "Mitogen-activated protein kinase kinase kinase kinase 5",
  "gene_symbol": "MAP4K5"
}